{
  "term_id": "UNKNOWN:0001",
  "gene_symbol": "CCDC159",
  "term_label": "Unknown molecular function",
  "gene_name": "Coiled-coil domain-containing protein 159",
  "gene": "UniProtKB:P0C7I6"
}